{
  "term_id": "GO:0005737",
  "gene": "UniProtKB:P02795",
  "gene_symbol": "MT2A",
  "gene_name": "Metallothionein-2",
  "term_label": "cytoplasm"
}